{
  "gene": "UniProtKB:P57721",
  "term_label": "regulation of transcription by RNA polymerase II",
  "gene_name": "Poly(rC)-binding protein 3",
  "gene_symbol": "PCBP3",
  "term_id": "GO:0006357"
}